multinuclear osteoclast differentiation [GO:0072674] (biological process) Also known as: multinuclear osteoclast formation, multinuclear osteoclast morphogenesis Relationships: is a type of osteoclast differentiation [GO:0030316] References: PMID:12713016 Sources: CL:0000779, GOC:mah Definition: The process in which a relatively unspecialized monocyte acquires the specialized features of a multinuclear osteoclast. An osteoclast is a specialized phagocytic cell associated with the absorption and removal of the mineralized matrix of bone tissue.